{
  "term_id": "UNKNOWN:0001",
  "gene": "UniProtKB:Q9Y3V2",
  "gene_name": "RWD domain-containing protein 3",
  "term_label": "Unknown molecular function",
  "gene_symbol": "RWDD3"
}